{
  "gene_symbol": "ZFAND2A",
  "gene_name": "AN1-type zinc finger protein 2A",
  "gene": "UniProtKB:Q8N6M9",
  "term_id": "GO:0045047",
  "term_label": "protein targeting to ER"
}